N-acylglucosamine 2-epimerase activity [GO:0050121] (molecular function) Also known as: GlcNAc 2-epimerase activity, N-acetyl-D-glucosamine 2-epimerase activity, N-acetylglucosamine 2-epimerase activity, N-acyl-D-glucosamine 2-epimerase activity, acylglucosamine 2-epimerase activity Relationships: is a type of GO:0016857 Sources: EC:5.1.3.8, MetaCyc:N-ACYLGLUCOSAMINE-2-EPIMERASE-RXN Definition: Catalysis of the reaction: N-acyl-D-glucosamine = N-acyl-D-mannosamine.